phthalate metabolic process [GO:0018963] (biological process) Relationships: is a type of GO:0019752; is a type of benzene-containing compound metabolic process [GO:0042537] Definition: The chemical reactions and pathways involving phthalate, the anion of phthalic acid. Phthalic acid diesters are used industrially in the production of a variety of household and consumer goods including plastic polymers, lubricating oils, and carriers for perfumes in cosmetics, while phthalic acid itself is used industrially as a plasticizer. Terephthalate is used in the synthesis of polyethylene terephthalate (polyethene terephthlate, abbreviated PET or PETE), a plastic polymer with many commercial uses. Also known as: phthalate metabolism, phthalic acid metabolic process, phthalic acid metabolism Subtypes: phthalate catabolic process [GO:0046239] Sources: UM-BBD_pathwayID:pth